purine nucleobase transport [GO:0006863] (biological process) Subtypes: adenine transport [GO:0015853], guanine transport [GO:0015854], hypoxanthine transport [GO:0035344], GO:0042906, purine nucleobase transmembrane transport [GO:1904823] Relationships: is a type of nucleobase transport [GO:0015851] Definition: The directed movement of purine bases, one of the two classes of nitrogen-containing ring compounds found in DNA and RNA, into, out of or within a cell, or between cells, by means of some agent such as a transporter or pore. Sources: ISBN:0198506732 Also known as: purine base transmembrane transport, purine base transport, purine transmembrane transport, purine transport